MHC class Ib protein complex [GO:0032398] (cellular component) Relationships: is a type of MHC protein complex [GO:0042611] Definition: A transmembrane protein complex composed of a MHC class Ib alpha chain and, in most cases, an invariant beta2-microglobin chain, and with or without a bound peptide or lipid antigen. Class Ib here refers to non-classical class I molecules, such as those of the CD1 or HLA-E gene families. References: PMID:15928678 Sources: GOC:add, ISBN:0781735149